{
  "gene": "UniProtKB:O00339",
  "term_label": "Unknown molecular function",
  "gene_name": "Matrilin-2",
  "gene_symbol": "MATN2",
  "term_id": "UNKNOWN:0001"
}